{
  "gene_symbol": "STYX",
  "term_id": "UNKNOWN:0001",
  "term_label": "Unknown molecular function",
  "gene": "UniProtKB:Q8WUJ0",
  "gene_name": "Serine_threonine_tyrosine-interacting protein"
}